{
  "gene": "UniProtKB:Q9BWE0",
  "term_id": "GO:0005634",
  "term_label": "nucleus",
  "gene_symbol": "REPIN1",
  "gene_name": "Replication initiator 1"
}